negative regulation of fever generation [GO:0031621] (biological process) Sources: GOC:add, GOC:dph, GOC:tb Relationships: is a type of negative regulation of acute inflammatory response [GO:0002674]; is_a regulation of fever generation [GO:0031620]; is a type of GO:0031651; negatively regulates GO:0001660 Definition: Any process that stops, prevents, or reduces the rate or extent of fever generation. Also known as: down regulation of fever, down-regulation of fever, downregulation of fever, negative regulation of pyrexia, inhibition of fever